{
  "gene_name": "Na(+)_H(+) exchange regulatory cofactor NHE-RF3",
  "gene": "UniProtKB:Q5T2W1",
  "gene_symbol": "PDZK1",
  "term_id": "GO:0043495",
  "term_label": "protein-membrane adaptor activity"
}